positive regulation of hindgut contraction [GO:0060450] (biological process) Relationships: is a type of regulation of hindgut contraction [GO:0043134]; is a type of positive regulation of smooth muscle contraction [GO:0045987]; is a type of positive regulation of digestive system process [GO:0060456]; positively regulates GO:0043133 Definition: Any process that increases the frequency, rate or extent of muscle contraction of the hindgut, the posterior part of the alimentary canal, including the rectum, and the large intestine. Sources: GOC:dph, GOC:tb